{
  "gene_name": "DNA helicase B",
  "gene": "UniProtKB:Q8NG08",
  "gene_symbol": "HELB",
  "term_id": "GO:0017116",
  "term_label": "single-stranded DNA helicase activity"
}